energy reserve metabolic process [GO:0006112] (biological process) Relationships: is a type of GO:0015980 Also known as: energy reserve metabolism Subtypes: glycogen metabolic process [GO:0005977] Sources: GOC:mah Definition: The chemical reactions and pathways by which a cell derives energy from stored compounds such as fats or glycogen.